{
  "gene": "UniProtKB:P00390",
  "term_id": "GO:0005829",
  "gene_name": "Glutathione reductase, mitochondrial",
  "gene_symbol": "GSR",
  "term_label": "cytosol"
}